{
  "term_label": "Unknown molecular function",
  "gene": "UniProtKB:Q99575",
  "term_id": "UNKNOWN:0001",
  "gene_symbol": "POP1",
  "gene_name": "Ribonucleases P_MRP protein subunit POP1"
}